{
  "gene_name": "Tectonin beta-propeller repeat-containing protein 2",
  "gene": "UniProtKB:O15040",
  "gene_symbol": "TECPR2",
  "term_id": "UNKNOWN:0001",
  "term_label": "Unknown molecular function"
}